alpha-1B adrenergic receptor binding [GO:0031692] (MF) Definition: Binding to an alpha-1B adrenergic receptor. Sources: GOC:mah, GOC:nln Also known as: alpha-1B adrenergic receptor ligand Relationships: is a type of GO:0031690